Mad-Max-mSin3A complex [GO:0070439] (cellular component) References: PMID:7889570 Definition: A transcriptional repressor complex that contains a heterodimer of the bHLH-ZIP proteins Mad and Max, plus mSin3A, a homolog of the yeast Sin3p. Relationships: is a type of RNA polymerase II transcription repressor complex [GO:0090571]